{
  "gene_name": "Placenta growth factor",
  "term_id": "GO:0060754",
  "term_label": "positive regulation of mast cell chemotaxis",
  "gene": "UniProtKB:P49763",
  "gene_symbol": "PGF"
}